lipase activator activity [GO:0060229] (molecular function) Subtypes: phospholipase activator activity [GO:0016004], lipoprotein lipase activator activity [GO:0060230] Definition: Binds to and increases the activity of a lipase, an enzyme that catalyzes of the hydrolysis of a lipid. Relationships: is a type of enzyme activator activity [GO:0008047]; positively regulates lipase activity [GO:0016298] Sources: GOC:BHF, GOC:dph, GOC:tb